{
  "gene": "UniProtKB:Q96NR3",
  "term_id": "GO:0045202",
  "term_label": "synapse",
  "gene_name": "Patched domain-containing protein 1",
  "gene_symbol": "PTCHD1"
}